{
  "term_label": "glutaminase activity",
  "term_id": "GO:0004359",
  "gene_name": "Glutaminase liver isoform, mitochondrial",
  "gene_symbol": "GLS2",
  "gene": "UniProtKB:Q9UI32"
}